{
  "term_id": "UNKNOWN:0001",
  "gene_name": "Pregnancy-specific beta-1-glycoprotein 8",
  "term_label": "Unknown molecular function",
  "gene_symbol": "PSG8",
  "gene": "UniProtKB:Q9UQ74"
}